response to muscle inactivity [GO:0014870] (biological process) Relationships: is a type of response to inactivity [GO:0014854] Definition: Any process that results in a change in state or activity of a cell or an organism (in terms of movement, secretion, enzyme production, gene expression, etc.) as a result of a muscle inactivity stimulus. Subtypes: GO:0014869, response to muscle inactivity involved in regulation of muscle adaptation [GO:0014877] Sources: GOC:mtg_muscle